negative regulation of L-proline biosynthetic process [GO:1902006] (biological process) Definition: Any process that stops, prevents or reduces the frequency, rate or extent of L-proline biosynthetic process. Also known as: negative regulation of proline biosynthetic process, down regulation of proline anabolism, down regulation of proline biosynthesis, down regulation of proline biosynthetic process, down regulation of proline formation, down regulation of proline synthesis, down-regulation of proline anabolism, down-regulation of proline biosynthesis, down-regulation of proline biosynthetic process, down-regulation of proline formation, down-regulation of proline synthesis, downregulation of proline anabolism, downregulation of proline biosynthesis, downregulation of proline biosynthetic process, downregulation of proline formation, downregulation of proline synthesis, inhibition of proline anabolism, inhibition of proline biosynthesis, inhibition of proline formation, inhibition of proline synthesis, negative regulation of proline anabolism, negative regulation of proline biosynthesis, negative regulation of proline formation, negative regulation of proline synthesis, inhibition of proline biosynthetic process References: PMID:23415322 Sources: GOC:TermGenie Relationships: is a type of negative regulation of small molecule metabolic process [GO:0062014]; is a type of GO:1902005; is a type of negative regulation of amino acid biosynthetic process [GO:2000283]; negatively regulates L-proline biosynthetic process [GO:0055129]